neuropeptide F receptor activity [GO:0042263] (molecular function) Relationships: is a type of neuropeptide receptor activity [GO:0008188] Also known as: NPF receptor activity References: PMID:21440021 Sources: GOC:bf, GOC:ma Definition: Combining with neuropeptide F and transmitting the signal within the cell to initiate a change in cell activity. Neuropeptide F is an arthropod peptide of more than 28 residues (typically 28-45) with a consensus C-terminal RxRFamide (commonly RPRFa, but also RVRFa. Note: Despite their naming, neuropeptide F (NPF) and short neuropeptide F (sNPF) are not closely related.